{
  "term_id": "GO:0005681",
  "gene": "UniProtKB:Q96E39",
  "gene_name": "RNA binding motif protein, X-linked-like-1",
  "term_label": "spliceosomal complex",
  "gene_symbol": "RBMXL1"
}